{
  "term_id": "GO:0061575",
  "gene": "UniProtKB:Q13319",
  "gene_name": "Cyclin-dependent kinase 5 activator 2",
  "gene_symbol": "CDK5R2",
  "term_label": "cyclin-dependent protein serine/threonine kinase activator activity"
}